{
  "gene": "UniProtKB:Q16548",
  "term_label": "mitochondrial outer membrane",
  "gene_name": "Bcl-2-related protein A1",
  "term_id": "GO:0005741",
  "gene_symbol": "BCL2A1"
}